capsular polysaccharide transport [GO:0015776] (biological process) Definition: The directed movement of capsular polysaccharides into, out of or within a cell, or between cells, by means of some agent such as a transporter or pore. Capsular polysaccharides make up the capsule, a protective structure surrounding some species of bacteria and fungi. Sources: GOC:ai Also known as: capsular-polysaccharide transport, capsule polysaccharide transport Relationships: is a type of polysaccharide transport [GO:0015774]